nucleosomal DNA binding [GO:0031492] (molecular function) Relationships: is_a chromatin DNA binding [GO:0031490]; is a type of nucleosome binding [GO:0031491] Sources: GOC:mah Definition: Binding to the DNA portion of a nucleosome.